symbiont-mediated suppression of host pro-inflammatory cytokine signaling [GO:0141173] (biological process) Definition: A process by which a symbiont inhibits or disrupts pro-inflammatory cytokine signaling in the host organism, either by disruption of production, sequesteration, or destruction of at least one component of the signaling pathway. Pro-inflammatory cytokines include: IL-1, IL-12, IL-18, TNF, IFN-gamma, and GM-CSF. The host is defined as the larger of the organisms involved in a symbiotic interaction. References: PMID:20008527, PMID:24508400, PMID:32117813 Also known as: negative regulation by symbiont of host pro-inflammatory cytokine production, suppression by symbiont of host pro-inflammatory cytokine production, symbiont-mediated degradation of host pro-inflammatory cytokine, suppression by symbiont of host pro-inflammatory cytokine secretion, symbiont-mediated sequestering of host pro-inflammatory cytokine, symbiont-mediated suppression of host pro-inflammatory cytokine production Relationships: is a type of GO:0075109